{
  "gene": "UniProtKB:P01241",
  "gene_symbol": "GH1",
  "term_id": "GO:0005179",
  "term_label": "hormone activity",
  "gene_name": "Somatotropin"
}